{
  "gene_symbol": "BTN2A2",
  "term_id": "GO:0005102",
  "gene": "UniProtKB:Q8WVV5",
  "gene_name": "Butyrophilin subfamily 2 member A2",
  "term_label": "signaling receptor binding"
}